peptidyl-lysine monomethylation [GO:0018026] (biological process) Sources: RESID:AA0076 Relationships: is_a peptidyl-lysine methylation [GO:0018022] Definition: The methylation of peptidyl-lysine to form peptidyl-N6-methyl-L-lysine.